regulation of reverse transcription [GO:1900268] (biological process) Definition: Any process that modulates the frequency, rate or extent of reverse transcription. Relationships: is a type of GO:2000278; regulates reverse transcription [GO:0001171] Subtypes: negative regulation of reverse transcription [GO:1900269], positive regulation of reverse transcription [GO:1900270] Sources: GOC:TermGenie